regulation of hematopoietic stem cell differentiation [GO:1902036] (biological process) Definition: Any process that modulates the frequency, rate or extent of hematopoietic stem cell differentiation. Relationships: is a type of GO:1901532; is a type of regulation of stem cell differentiation [GO:2000736]; regulates GO:0060218 Subtypes: negative regulation of hematopoietic stem cell differentiation [GO:1902037], GO:1902038 Also known as: regulation of haematopoietic stem cell differentiation, regulation of haemopoietic stem cell differentiation, regulation of hemopoietic stem cell differentiation References: PMID:23403623 Sources: GOC:TermGenie